{
  "term_id": "GO:0015280",
  "gene_symbol": "ASIC1",
  "term_label": "ligand-gated sodium channel activity",
  "gene_name": "Acid-sensing ion channel 1",
  "gene": "UniProtKB:P78348"
}